{
  "term_id": "GO:0006564",
  "gene_symbol": "PSPH",
  "gene": "UniProtKB:P78330",
  "gene_name": "Phosphoserine phosphatase",
  "term_label": "L-serine biosynthetic process"
}